negative regulation of smoothened signaling pathway involved in ventral spinal cord patterning [GO:0021914] (biological process) Definition: Any process that stops, prevents, or reduces the frequency, rate or extent of smoothened signaling that is involved in the patterns of cell differentiation in the ventral spinal cord. Relationships: is_a negative regulation of smoothened signaling pathway [GO:0045879]; BFO_0000050 spinal cord dorsal/ventral patterning [GO:0021513]; negatively regulates smoothened signaling pathway involved in ventral spinal cord patterning [GO:0021910] References: PMID:11262869 Sources: GOC:cls, GOC:dgh, GOC:dph, GOC:jid, GOC:tb Also known as: down regulation of smoothened signaling pathway in ventral spinal cord patterning, down-regulation of smoothened signaling pathway in ventral spinal cord patterning, downregulation of smoothened signaling pathway in ventral spinal cord patterning, negative regulation of hedgehog signaling pathway involved in ventral spinal cord patterning, negative regulation of hh signaling pathway involved in ventral spinal cord patterning, negative regulation of smoothened signalling pathway in ventral spinal cord patterning, inhibition of smoothened signaling pathway in ventral spinal cord patterning